RNA splicing, via endonucleolytic cleavage and ligation [GO:0000394] (biological process) Subtypes: tRNA splicing, via endonucleolytic cleavage and ligation [GO:0006388], mRNA splicing, via endonucleolytic cleavage and ligation [GO:0070054] Definition: Splicing of RNA via recognition of the folded RNA structure that brings the 5' and 3' splice sites into proximity and cleavage of the RNA at both the 3' and 5' splice sites by an endonucleolytic mechanism, followed by ligation of the exons. Relationships: is a type of GO:0008380 Note: Note that while typically associated with tRNA splicing, this mechanism of splicing is known to be used for some non-tRNA substrates, e.g. HAC1 (YFL031W) in S. cerevisiae and an intron in the 23S rRNA of the Archaeal species Desulfurococcus mobilis. Also known as: mRNA splicing Sources: GOC:krc, ISBN:0879695897